{
  "gene_name": "Transcription factor GATA-4",
  "gene_symbol": "GATA4",
  "term_id": "GO:0005634",
  "gene": "UniProtKB:P43694",
  "term_label": "nucleus"
}